{
  "gene_name": "Neurturin",
  "gene_symbol": "NRTN",
  "gene": "UniProtKB:Q99748",
  "term_id": "GO:0035860",
  "term_label": "glial cell-derived neurotrophic factor receptor signaling pathway"
}